{
  "gene_name": "F-box_SPRY domain-containing protein 1",
  "term_label": "synapse assembly involved in innervation",
  "gene_symbol": "FBXO45",
  "gene": "UniProtKB:P0C2W1",
  "term_id": "GO:0060386"
}